{
  "gene_name": "NAD-dependent protein deacetylase sirtuin-1",
  "term_label": "DNA damage response",
  "gene": "UniProtKB:Q96EB6",
  "gene_symbol": "SIRT1",
  "term_id": "GO:0006974"
}